{
  "term_label": "RNA polymerase II transcription regulatory region sequence-specific DNA binding",
  "term_id": "GO:0000977",
  "gene_symbol": "ZFP41",
  "gene": "UniProtKB:Q8N8Y5",
  "gene_name": "Zinc finger protein 41 homolog"
}